{
  "term_id": "GO:0048013",
  "gene_symbol": "EPHB2",
  "gene": "UniProtKB:P29323",
  "gene_name": "Ephrin type-B receptor 2",
  "term_label": "ephrin receptor signaling pathway"
}